{
  "gene": "UniProtKB:P13765",
  "term_id": "GO:0042613",
  "gene_symbol": "HLA-DOB",
  "term_label": "MHC class II protein complex",
  "gene_name": "HLA class II histocompatibility antigen, DO beta chain"
}